{
  "term_label": "epidermal growth factor receptor signaling pathway",
  "gene_symbol": "IQGAP1",
  "gene": "UniProtKB:P46940",
  "gene_name": "Ras GTPase-activating-like protein IQGAP1",
  "term_id": "GO:0007173"
}